proteinase activated receptor binding [GO:0031871] (molecular function) Sources: GOC:mah, GOC:nln Relationships: is a type of G protein-coupled receptor binding [GO:0001664] Subtypes: type 1 proteinase activated receptor binding [GO:0031872], GO:0031873, type 3 proteinase activated receptor binding [GO:0031874], type 4 proteinase activated receptor binding [GO:0031875] Also known as: proteinase activated receptor ligand Definition: Binding to a proteinase activated receptor.